{
  "gene_name": "T cell receptor gamma constant 1",
  "term_label": "Unknown biological process",
  "gene": "UniProtKB:P0CF51",
  "gene_symbol": "TRGC1",
  "term_id": "UNKNOWN:0002"
}